{
  "gene_symbol": "GLB1L",
  "gene_name": "Beta-galactosidase-1-like protein",
  "gene": "UniProtKB:Q6UWU2",
  "term_label": "vacuole",
  "term_id": "GO:0005773"
}